{
  "term_label": "microfilament motor activity",
  "term_id": "GO:0000146",
  "gene_name": "Myosin-4",
  "gene_symbol": "MYH4",
  "gene": "UniProtKB:Q9Y623"
}